{
  "gene": "UniProtKB:Q9UKW4",
  "term_label": "plasma membrane",
  "gene_name": "Guanine nucleotide exchange factor VAV3",
  "gene_symbol": "VAV3",
  "term_id": "GO:0005886"
}